fructoselysine metabolic process [GO:0030393] (biological process) Also known as: fructoselysine metabolism Relationships: is a type of carboxylic acid metabolic process [GO:0019752]; is a type of fructosamine metabolic process [GO:0030389] Subtypes: fructoselysine catabolic process [GO:1901281], fructoselysine biosynthetic process [GO:1901282] Definition: The chemical reactions and pathways involving fructoselysine, a fructose molecule containing a lysine group in place of a hydroxyl group. Sources: GOC:ai